{
  "term_label": "Unknown cellular component",
  "gene_symbol": "GSTM5",
  "gene_name": "Glutathione S-transferase Mu 5",
  "gene": "UniProtKB:P46439",
  "term_id": "UNKNOWN:0003"
}